alkene monooxygenase activity [GO:0018645] (molecular function) Also known as: alkene epoxygenase activity, alkene,NADH:oxygen oxidoreductase activity Definition: Catalysis of the reaction: propene + NADH + H+ + O2 = 1,2-epoxypropane + NAD+ + H2O. Relationships: is a type of oxidoreductase activity, acting on paired donors, with incorporation or reduction of molecular oxygen, NAD(P)H as one donor, and incorporation of one atom of oxygen [GO:0016709] Sources: EC:1.14.13.69